raffinose metabolic process [GO:0033530] (biological process) Definition: The chemical reactions and pathways involving raffinose, the trisaccharide beta-D-fructofuranosyl alpha-D-galactopyranosyl-(1->6)-alpha-D-glucopyranoside. Sources: GOC:mah Also known as: raffinose metabolism Relationships: is a type of oligosaccharide metabolic process [GO:0009311] Subtypes: raffinose biosynthetic process [GO:0033529], raffinose catabolic process [GO:0034484] Regulation: regulated by regulation of raffinose metabolic process [GO:0080091]